{
  "term_id": "GO:0050830",
  "gene_name": "Peptidoglycan recognition protein 4",
  "gene_symbol": "PGLYRP4",
  "term_label": "defense response to Gram-positive bacterium",
  "gene": "UniProtKB:Q96LB8"
}